{
  "gene_symbol": "STX8",
  "term_label": "vesicle docking",
  "term_id": "GO:0048278",
  "gene_name": "Syntaxin-8",
  "gene": "UniProtKB:Q9UNK0"
}